{
  "gene_name": "Mitochondrial coenzyme A transporter SLC25A42",
  "gene": "UniProtKB:Q86VD7",
  "gene_symbol": "SLC25A42",
  "term_label": "Unknown cellular component",
  "term_id": "UNKNOWN:0003"
}